{
  "gene_symbol": "CYB5R2",
  "term_id": "GO:0005739",
  "gene_name": "NADH-cytochrome b5 reductase 2",
  "term_label": "mitochondrion",
  "gene": "UniProtKB:Q6BCY4"
}